{
  "gene_symbol": "SPRY4",
  "term_id": "GO:0040037",
  "gene_name": "Protein sprouty homolog 4",
  "term_label": "negative regulation of fibroblast growth factor receptor signaling pathway",
  "gene": "UniProtKB:Q9C004"
}